{
  "gene_name": "Matrix metalloproteinase-24",
  "gene": "UniProtKB:Q9Y5R2",
  "term_id": "GO:0030198",
  "gene_symbol": "MMP24",
  "term_label": "extracellular matrix organization"
}